{
  "gene": "UniProtKB:Q9HD20",
  "gene_symbol": "ATP13A1",
  "gene_name": "Endoplasmic reticulum transmembrane helix translocase",
  "term_label": "P-type ion transporter activity",
  "term_id": "GO:0015662"
}